{
  "gene_name": "[Pyruvate dehydrogenase (acetyl-transferring)] kinase isozyme 4, mitochondrial",
  "gene_symbol": "PDK4",
  "term_id": "GO:0005739",
  "term_label": "mitochondrion",
  "gene": "UniProtKB:Q16654"
}